{
  "gene_symbol": "YOD1",
  "gene_name": "Ubiquitin thioesterase OTU1",
  "term_label": "ERAD pathway",
  "gene": "UniProtKB:Q5VVQ6",
  "term_id": "GO:0036503"
}